{
  "term_label": "histone methyltransferase complex",
  "term_id": "GO:0035097",
  "gene_name": "Histone-lysine N-methyltransferase 2B",
  "gene_symbol": "KMT2B",
  "gene": "UniProtKB:Q9UMN6"
}